tRNA (guanine-N7)-methylation [GO:0106004] (biological process) Relationships: is a type of tRNA methylation [GO:0030488]; is a type of RNA (guanine-N7)-methylation [GO:0036265] Definition: The process whereby a guanine in a tRNA is methylated at the N7 position of guanine. References: PMID:17382321 Sources: GOC:hjd